{
  "term_id": "UNKNOWN:0001",
  "term_label": "Unknown molecular function",
  "gene_name": "T cell receptor alpha variable 4",
  "gene": "UniProtKB:A0A0B4J268",
  "gene_symbol": "TRAV4"
}